{
  "gene_name": "Cardiotrophin-1",
  "gene": "UniProtKB:Q16619",
  "term_id": "GO:0005125",
  "gene_symbol": "CTF1",
  "term_label": "cytokine activity"
}